{
  "gene_name": "Heat shock protein beta-2",
  "term_id": "GO:0043066",
  "gene_symbol": "HSPB2",
  "term_label": "negative regulation of apoptotic process",
  "gene": "UniProtKB:Q16082"
}